{
  "term_label": "G protein-coupled peptide receptor activity",
  "gene": "UniProtKB:Q13324",
  "term_id": "GO:0008528",
  "gene_symbol": "CRHR2",
  "gene_name": "Corticotropin-releasing factor receptor 2"
}